propanediol dehydratase activity [GO:0050215] (molecular function) Also known as: 1,2-propanediol dehydratase activity, DL-1,2-propanediol hydro-lyase activity, adenosylcobalamin-dependent diol dehydratase activity, coenzyme B12-dependent diol dehydrase activity, diol dehydrase activity, diol dehydratase activity, dioldehydratase activity, meso-2,3-butanediol dehydrase activity, propane-1,2-diol hydro-lyase (propanal-forming), propane-1,2-diol hydro-lyase activity, propanediol dehydrase activity Relationships: is a type of hydro-lyase activity [GO:0016836] Definition: Catalysis of the reaction: propane-1,2-diol = H2O + propanal. Sources: EC:4.2.1.28, RHEA:14569